L-cysteine catabolic process to pyruvate [GO:0019450] (biological process) Relationships: is a type of pyruvate metabolic process [GO:0006090]; is a type of L-cysteine catabolic process [GO:0019448] Sources: GOC:go_curators Subtypes: L-cysteine catabolic process to pyruvate, using cysteine dioxygenase [GO:0019451] Also known as: L-cysteine breakdown to pyruvate, L-cysteine degradation to pyruvate Definition: The chemical reactions and pathways resulting in the breakdown of L-cysteine into other compounds, including pyruvate.